{
  "gene": "UniProtKB:O43812",
  "term_label": "regulation of transcription by RNA polymerase II",
  "gene_name": "Double homeobox protein 1",
  "gene_symbol": "DUX1",
  "term_id": "GO:0006357"
}